{
  "gene_name": "Mitochondrial genome maintenance exonuclease 1",
  "term_label": "single-stranded DNA exodeoxyribonuclease activity",
  "gene": "UniProtKB:Q9BQP7",
  "term_id": "GO:0008297",
  "gene_symbol": "MGME1"
}